tetrahydrobiopterin binding [GO:0034617] (molecular function) Also known as: BH4 binding, H4biopterin binding, sapropterin binding Definition: Binding to a tetrahydrobiopterin, 5,6,7,8-tetrahydrobiopterin or a derivative thereof; tetrahydrobiopterins are enzyme cofactors that carry electrons in redox reactions. Sources: GOC:BHF, GOC:mah, GOC:rl Subtypes: GO:0071576 Relationships: is a type of GO:0005488